alpha-sialidase activity [GO:0016997] (molecular function) Sources: GOC:mah Subtypes: exo-alpha-sialidase activity [GO:0004308], endo-alpha-(2,8)-sialidase activity [GO:0016996], GO:0052791 Definition: Catalysis of the hydrolysis of alpha-glycosidic linkages in oligo- or poly(sialic) acids. Relationships: is a type of GO:0004553